{
  "gene_symbol": "CDC25B",
  "gene": "UniProtKB:P30305",
  "gene_name": "M-phase inducer phosphatase 2",
  "term_id": "GO:0000086",
  "term_label": "G2/M transition of mitotic cell cycle"
}